trifid subdivision of terminal units involved in ureteric bud branching [GO:0060679] (biological process) Relationships: is a type of morphogenesis of an epithelium [GO:0002009]; is part of branching involved in ureteric bud morphogenesis [GO:0001658] Definition: The process in which a ureteric bud splits into three units at its end. References: PMID:16916378 Sources: GOC:dph